extrinsic component of lumenal side of plastid thylakoid membrane [GO:0035450] (cellular component) Subtypes: extrinsic component of stromal side of plastid inner membrane [GO:0035454] Sources: GOC:bf, GOC:dos Definition: The component of a plastid thylakoid membrane consisting of gene products and protein complexes that are loosely bound to its lumenal surface, but not integrated into the hydrophobic region. Relationships: is_a extrinsic component of plastid thylakoid membrane [GO:0035449]; is a type of extrinsic component of plastid inner membrane [GO:0035453]; is part of stromal side of plastid inner membrane [GO:0098570] Also known as: extrinsic to lumenal leaflet of plastid thylakoid membrane, peripheral to lumenal side of plastid thylakoid membrane, extrinsic to lumenal side of plastid thylakoid membrane